{
  "gene": "UniProtKB:Q8IWV1",
  "term_label": "immune response",
  "gene_symbol": "LAX1",
  "term_id": "GO:0006955",
  "gene_name": "Lymphocyte transmembrane adapter 1"
}